negative regulation of blood pressure [GO:0045776] (biological process) Sources: GOC:go_curators, GOC:mtg_cardio Subtypes: negative regulation of systemic arterial blood pressure [GO:0003085] Relationships: is a type of regulation of blood pressure [GO:0008217] Definition: Any process in which the force of blood traveling through the circulatory system is decreased. Also known as: down regulation of blood pressure, down-regulation of blood pressure, downregulation of blood pressure, inhibition of blood pressure